antibacterial innate immune response [GO:0140367] (biological process) References: PMID:16177355, PMID:23006328 Definition: An defense response against a bacteria mediated through an innate immune response. An innate immune response is mediated by germline encoded components that directly recognize components of potential pathogens. Relationships: is a type of defense response to bacterium [GO:0042742]; is a type of innate immune response [GO:0045087]